dsDNA-RNA triple helix-forming chromatin adaptor activity [GO:0141180] (MF) Definition: A chromatin-protein adaptor activity that bridges dsDNA and chromatin proteins to bring regions of a chromosome in proximity. The DNA:DNA:RNA triple-helical structure is formed non-Watson-Crick base-pairing. References: PMID:35412350 Relationships: is a type of GO:0140463; is a type of sequence-specific double-stranded DNA binding [GO:1990837]